aromatic amino acid transmembrane transporter activity [GO:0015173] (molecular function) Subtypes: L-histidine transmembrane transporter activity [GO:0005290], GO:0005302, GO:0015192, L-tryptophan transmembrane transporter activity [GO:0015196], aromatic amino acid:proton symporter activity [GO:0015494] Also known as: aromatic amino acid transporter activity, hydroxy/aromatic amino acid permease activity, valine/tyrosine/tryptophan permease activity Sources: GOC:ai, GOC:mtg_transport, ISBN:0815340729 Relationships: is a type of carboxylic acid transmembrane transporter activity [GO:0046943]; is part of aromatic amino acid transport [GO:0015801] Definition: Enables the transfer of aromatic amino acids from one side of a membrane to the other. Aromatic amino acids have an aromatic ring.